{
  "term_label": "Unknown biological process",
  "gene_name": "Keratin-associated protein 5-10",
  "term_id": "UNKNOWN:0002",
  "gene": "UniProtKB:Q6L8G5",
  "gene_symbol": "KRTAP5-10"
}